{
  "term_label": "nuclear envelope",
  "gene": "UniProtKB:O15504",
  "gene_name": "Nucleoporin NUP42",
  "term_id": "GO:0005635",
  "gene_symbol": "NUP42"
}